{
  "gene_symbol": "CAPG",
  "term_label": "phosphatidylinositol-4,5-bisphosphate binding",
  "gene": "UniProtKB:P40121",
  "term_id": "GO:0005546",
  "gene_name": "Macrophage-capping protein"
}